regulation of response to oxidative stress [GO:1902882] (biological process) Definition: Any process that modulates the frequency, rate or extent of response to oxidative stress. References: PMID:16899554 Sources: GOC:TermGenie, GOC:kmv, GO_REF:0000058 Relationships: is a type of regulation of response to stress [GO:0080134]; regulates response to oxidative stress [GO:0006979] Subtypes: regulation of cellular response to oxidative stress [GO:1900407], regulation of response to reactive oxygen species [GO:1901031], negative regulation of response to oxidative stress [GO:1902883], GO:1902884